leucokinin receptor activity [GO:0042071] (molecular function) References: PMID:2716741 Sources: GOC:mah, GOC:signaling Definition: Combining with a leucokinin, any of several octapeptide hormones found in insects, and transmitting the signal to initiate a change in cell activity. Relationships: is a type of signaling receptor activity [GO:0038023]; is part of hormone-mediated signaling pathway [GO:0009755]